{
  "term_id": "GO:0034045",
  "gene": "UniProtKB:Q8IYT8",
  "gene_name": "Serine_threonine-protein kinase ULK2",
  "term_label": "phagophore assembly site membrane",
  "gene_symbol": "ULK2"
}